{
  "gene_name": "Zinc finger protein 789",
  "term_label": "regulation of transcription by RNA polymerase II",
  "term_id": "GO:0006357",
  "gene_symbol": "ZNF789",
  "gene": "UniProtKB:Q5FWF6"
}